{
  "gene": "UniProtKB:P50479",
  "gene_name": "PDZ and LIM domain protein 4",
  "term_label": "muscle alpha-actinin binding",
  "term_id": "GO:0051371",
  "gene_symbol": "PDLIM4"
}